negative regulation of odontogenesis [GO:0042483] (biological process) Also known as: down regulation of odontogenesis, down-regulation of odontogenesis, downregulation of odontogenesis, negative regulation of tooth development, inhibition of odontogenesis, negative regulation of odontogenesis of calcareous or chitinous tooth Subtypes: negative regulation of odontogenesis of dentin-containing tooth [GO:0042489] Definition: Any process that stops, prevents, or reduces the frequency, rate or extent of the formation and development of a tooth or teeth. Sources: GOC:jl Relationships: is a type of regulation of odontogenesis [GO:0042481]; is a type of GO:0110111; negatively regulates odontogenesis [GO:0042476]